{
  "gene": "UniProtKB:P56134",
  "gene_symbol": "ATP5MF",
  "term_id": "GO:0045259",
  "gene_name": "ATP synthase subunit f, mitochondrial",
  "term_label": "proton-transporting ATP synthase complex"
}